{
  "term_id": "GO:0016020",
  "gene_name": "V-set and transmembrane domain-containing protein 2-like protein",
  "gene_symbol": "VSTM2L",
  "term_label": "membrane",
  "gene": "UniProtKB:Q96N03"
}